{
  "gene_symbol": "PTAFR",
  "term_label": "Unknown cellular component",
  "gene": "UniProtKB:P25105",
  "term_id": "UNKNOWN:0003",
  "gene_name": "Platelet-activating factor receptor"
}